{
  "term_id": "GO:0003700",
  "gene_symbol": "ZBED3",
  "gene": "UniProtKB:Q96IU2",
  "term_label": "DNA-binding transcription factor activity",
  "gene_name": "Zinc finger BED domain-containing protein 3"
}